{
  "gene_name": "Zinc finger protein 26",
  "term_id": "UNKNOWN:0002",
  "gene_symbol": "ZNF26",
  "term_label": "Unknown biological process",
  "gene": "UniProtKB:P17031"
}